{
  "gene": "UniProtKB:O43684",
  "gene_symbol": "BUB3",
  "term_label": "ubiquitin binding",
  "term_id": "GO:0043130",
  "gene_name": "Mitotic checkpoint protein BUB3"
}